{
  "gene": "UniProtKB:P48723",
  "term_id": "GO:0042026",
  "gene_name": "Heat shock 70 kDa protein 13",
  "gene_symbol": "HSPA13",
  "term_label": "protein refolding"
}